{
  "gene_name": "Zinc finger protein 611",
  "term_label": "DNA-binding transcription factor activity, RNA polymerase II-specific",
  "term_id": "GO:0000981",
  "gene_symbol": "ZNF611",
  "gene": "UniProtKB:Q8N823"
}